{
  "term_id": "GO:0016020",
  "term_label": "membrane",
  "gene_symbol": "UPK3B",
  "gene_name": "Uroplakin-3b",
  "gene": "UniProtKB:Q9BT76"
}